{
  "term_id": "GO:0005737",
  "gene_symbol": "OAZ1",
  "term_label": "cytoplasm",
  "gene": "UniProtKB:P54368",
  "gene_name": "Ornithine decarboxylase antizyme 1"
}